{
  "gene_name": "Ubiquitin-conjugating enzyme E2 variant 2",
  "gene_symbol": "UBE2V2",
  "term_id": "GO:0005634",
  "gene": "UniProtKB:Q15819",
  "term_label": "nucleus"
}